{
  "gene": "UniProtKB:P51153",
  "gene_name": "Ras-related protein Rab-13",
  "gene_symbol": "RAB13",
  "term_id": "GO:0030140",
  "term_label": "trans-Golgi network transport vesicle"
}